{
  "term_label": "mRNA binding",
  "gene_symbol": "THOC2",
  "gene": "UniProtKB:Q8NI27",
  "term_id": "GO:0003729",
  "gene_name": "THO complex subunit 2"
}